{
  "gene_name": "FXYD domain-containing ion transport regulator 5",
  "term_label": "positive regulation of sodium ion export across plasma membrane",
  "gene_symbol": "FXYD5",
  "gene": "UniProtKB:Q96DB9",
  "term_id": "GO:1903278"
}